{
  "gene_symbol": "LINC01554",
  "term_label": "Unknown molecular function",
  "gene": "UniProtKB:Q52M75",
  "term_id": "UNKNOWN:0001",
  "gene_name": "Putative uncharacterized protein encoded by LINC01554"
}